negative regulation of nucleotide biosynthetic process [GO:0030809] (biological process) Definition: Any process that stops, prevents, or reduces the frequency, rate or extent of the chemical reactions and pathways resulting in the formation of nucleotides. Sources: GOC:mah Also known as: down regulation of nucleotide biosynthetic process, down-regulation of nucleotide biosynthetic process, downregulation of nucleotide biosynthetic process, negative regulation of nucleotide anabolism, negative regulation of nucleotide biosynthesis, negative regulation of nucleotide formation, negative regulation of nucleotide synthesis, inhibition of nucleotide biosynthetic process Relationships: is a type of GO:0009890; is a type of regulation of nucleotide biosynthetic process [GO:0030808]; is a type of negative regulation of nucleotide metabolic process [GO:0045980]; negatively regulates nucleotide biosynthetic process [GO:0009165] Subtypes: negative regulation of purine nucleotide biosynthetic process [GO:1900372], negative regulation of pyrimidine nucleotide biosynthetic process [GO:1900398]